{
  "gene_name": "Lysophospholipid acyltransferase LPCAT4",
  "term_label": "endoplasmic reticulum",
  "gene_symbol": "LPCAT4",
  "gene": "UniProtKB:Q643R3",
  "term_id": "GO:0005783"
}